{
  "term_id": "UNKNOWN:0002",
  "term_label": "Unknown biological process",
  "gene": "UniProtKB:Q9Y6N3",
  "gene_symbol": "CLCA3P",
  "gene_name": "Calcium-activated chloride channel regulator family member 3"
}